{
  "term_label": "BLOC-1 complex",
  "gene_name": "Biogenesis of lysosome-related organelles complex 1 subunit 1",
  "gene_symbol": "BLOC1S1",
  "term_id": "GO:0031083",
  "gene": "UniProtKB:P78537"
}